embryonic appendage morphogenesis [GO:0035113] (biological process) Definition: The process, occurring in the embryo, by which the anatomical structures of the appendage are generated and organized. An appendage is an organ or part that is attached to the trunk of an organism, such as a limb or a branch. Sources: ISBN:0582227089 Relationships: is a type of GO:0035107; is_a embryonic morphogenesis [GO:0048598] Subtypes: GO:0030326, embryonic pectoral fin morphogenesis [GO:0035118], embryonic pelvic fin morphogenesis [GO:0035119], embryonic medial fin morphogenesis [GO:0035122]